positive regulation of ectoderm development [GO:2000385] (BP) Sources: GOC:BHF Relationships: is_a positive regulation of developmental process [GO:0051094]; is a type of GO:2000383; positively regulates ectoderm development [GO:0007398] Definition: Any process that activates or increases the frequency, rate or extent of ectoderm development.